{
  "gene": "UniProtKB:Q8NHE4",
  "gene_name": "V-type proton ATPase subunit e 2",
  "term_label": "vacuolar proton-transporting V-type ATPase, V0 domain",
  "term_id": "GO:0000220",
  "gene_symbol": "ATP6V0E2"
}